{
  "term_id": "GO:0005085",
  "term_label": "guanyl-nucleotide exchange factor activity",
  "gene_name": "Engulfment and cell motility protein 2",
  "gene_symbol": "ELMO2",
  "gene": "UniProtKB:Q96JJ3"
}